{
  "gene_symbol": "NR2E3",
  "gene": "UniProtKB:Q9Y5X4",
  "term_label": "nuclear receptor activity",
  "gene_name": "Photoreceptor-specific nuclear receptor",
  "term_id": "GO:0004879"
}